morula development [GO:0014000] (biological process) References: PMID:37935903, PMID:38386558, PMID:39361745 Relationships: is a type of GO:0009790 Definition: The process whose specific outcome is the progression of the morula over time. The morula is a spherical embryonic mass of blastomeres formed before the blastula and resulting from cleavage of the fertilized ovum.